white fat cell differentiation involved in mammary gland fat development [GO:0060642] (biological process) References: PMID:12558599 Sources: GOC:dph Relationships: is_a white fat cell differentiation [GO:0050872]; BFO_0000050 mammary gland fat development [GO:0060611] Definition: The process in which a preadipocyte acquires specialized features of a white adipocyte of the mammary gland. White adipocytes have cytoplasmic lipids arranged in a unique vacuole.